{
  "gene_name": "BOS complex subunit NOMO3",
  "gene": "UniProtKB:P69849",
  "term_id": "GO:0005789",
  "term_label": "endoplasmic reticulum membrane",
  "gene_symbol": "NOMO3"
}